{
  "gene_name": "Calcium-binding protein 39",
  "gene": "UniProtKB:Q9Y376",
  "term_id": "GO:0043539",
  "term_label": "protein serine/threonine kinase activator activity",
  "gene_symbol": "CAB39"
}